phosphogluconate dehydratase activity [GO:0004456] (molecular function) Definition: Catalysis of the reaction: 6-phospho-D-gluconate = 2-dehydro-3-deoxy-6-phospho-D-gluconate + H2O. Sources: EC:4.2.1.12, RHEA:17277 Also known as: 6-phospho-D-gluconate hydro-lyase (2-dehydro-3-deoxy-6-phospho-D-gluconate-forming), 6-phospho-D-gluconate hydro-lyase activity, 6-phosphogluconate dehydrase activity, 6-phosphogluconate dehydratase activity, 6-phosphogluconic dehydrase activity, gluconate 6-phosphate dehydratase activity, gluconate-6-phosphate dehydratase activity Relationships: is a type of hydro-lyase activity [GO:0016836]